{
  "term_label": "epithelial cell differentiation involved in prostate gland development",
  "term_id": "GO:0060742",
  "gene": "UniProtKB:P07602",
  "gene_symbol": "PSAP",
  "gene_name": "Prosaposin"
}